{
  "gene": "UniProtKB:Q9HBG7",
  "gene_symbol": "LY9",
  "term_label": "immune response",
  "term_id": "GO:0006955",
  "gene_name": "T-lymphocyte surface antigen Ly-9"
}